{
  "gene": "UniProtKB:Q12912",
  "gene_symbol": "IRAG2",
  "term_id": "UNKNOWN:0002",
  "term_label": "Unknown biological process",
  "gene_name": "Inositol 1,4,5-triphosphate receptor associated 2"
}